steroid hormone receptor complex assembly [GO:0006463] (biological process) Relationships: is a type of GO:0065003 Definition: The aggregation, arrangement and bonding together of a set of components to form a steroid hormone receptor complex, an intracellular receptor that binds steroid hormones. The complex is often a dimer, and forms after the steroid has bound the receptor. Sources: GOC:jl, Wikipedia:Steroid_hormone_receptor